ascending aorta development [GO:0035905] (biological process) Relationships: is a type of anatomical structure development [GO:0048856]; is part of GO:0035904 Sources: GOC:bf, GOC:dgh, MA:0002570, UBERON:0001496, Wikipedia:Ascending_aorta Definition: The progression of the ascending aorta over time, from its initial formation to the mature structure. The ascending aorta is the portion of the aorta in a two-pass circulatory system that lies between the heart and the arch of aorta. In a two-pass circulatory system blood passes twice through the heart to supply the body once.